{
  "gene": "UniProtKB:A0A087WSX0",
  "term_label": "Unknown molecular function",
  "gene_symbol": "IGLV5-45",
  "gene_name": "Immunoglobulin lambda variable 5-45",
  "term_id": "UNKNOWN:0001"
}